{
  "term_label": "Unknown cellular component",
  "term_id": "UNKNOWN:0003",
  "gene_symbol": "ZNF579",
  "gene": "UniProtKB:Q8NAF0",
  "gene_name": "Zinc finger protein 579"
}